{
  "term_label": "high-density lipoprotein particle remodeling",
  "term_id": "GO:0034375",
  "gene_symbol": "LPL",
  "gene_name": "Lipoprotein lipase",
  "gene": "UniProtKB:P06858"
}